{
  "term_id": "GO:0016567",
  "gene_symbol": "RNF115",
  "gene": "UniProtKB:Q9Y4L5",
  "term_label": "protein ubiquitination",
  "gene_name": "E3 ubiquitin-protein ligase RNF115"
}